[acyl-carrier-protein] S-acetyltransferase activity [GO:0004313] (molecular function) Also known as: ACAT activity, ACP S-acetyltransferase activity, [acyl-carrier protein] S-acetyltransferase activity, ACP acetyltransferase activity, ACPacetyltransferase activity, acetyl coenzyme A-acyl-carrier-protein transacylase activity, acetyl-CoA:acyl-carrier-protein S-acetyltransferase activity, acyl-carrier-protein S-acetyltransferase activity, acyl-carrier-protein acetyltransferase activity, acyl-carrier-proteinacetyltransferase activity Definition: Catalysis of the reaction: acetyl-CoA + [acyl-carrier protein] = CoA + acetyl-[acyl-carrier protein]. Sources: RHEA:41788 Relationships: is a type of S-acetyltransferase activity [GO:0016418]